{
  "term_id": "GO:0045893",
  "term_label": "positive regulation of DNA-templated transcription",
  "gene": "UniProtKB:Q9Y463",
  "gene_symbol": "DYRK1B",
  "gene_name": "Dual specificity tyrosine-phosphorylation-regulated kinase 1B"
}